mitotic chromosome centromere condensation [GO:1990893] (BP) Definition: The cell cycle process in which centromere chromatin structure is compacted prior to and during mitosis. References: PMID:21633354 Also known as: mitotic chromosome condensation at kinetochore Relationships: is a type of GO:0007076